{
  "term_id": "GO:0007186",
  "term_label": "G protein-coupled receptor signaling pathway",
  "gene": "UniProtKB:Q8NGU9",
  "gene_symbol": "GPR150",
  "gene_name": "Probable G-protein coupled receptor 150"
}